{
  "gene_name": "Phospholipid scramblase 3",
  "term_label": "phospholipid scramblase activity",
  "term_id": "GO:0017128",
  "gene_symbol": "PLSCR3",
  "gene": "UniProtKB:Q9NRY6"
}